{
  "term_id": "GO:0044458",
  "gene_name": "Jouberin",
  "term_label": "motile cilium assembly",
  "gene": "UniProtKB:Q8N157",
  "gene_symbol": "AHI1"
}